{
  "term_label": "cell-cell signaling",
  "gene_symbol": "GJA1",
  "term_id": "GO:0007267",
  "gene": "UniProtKB:P17302",
  "gene_name": "Gap junction alpha-1 protein"
}